{
  "gene": "UniProtKB:A2PYH4",
  "term_label": "nucleus",
  "gene_symbol": "HFM1",
  "term_id": "GO:0005634",
  "gene_name": "Probable ATP-dependent DNA helicase HFM1"
}